{
  "term_id": "UNKNOWN:0001",
  "gene": "UniProtKB:P56715",
  "gene_symbol": "RP1",
  "gene_name": "Oxygen-regulated protein 1",
  "term_label": "Unknown molecular function"
}